{
  "term_label": "RNA binding",
  "gene_name": "Probable ATP-dependent RNA helicase DHX35",
  "gene": "UniProtKB:Q9H5Z1",
  "term_id": "GO:0003723",
  "gene_symbol": "DHX35"
}